{
  "term_label": "regulation of transcription by RNA polymerase II",
  "gene_name": "Homeobox protein Hox-A7",
  "gene": "UniProtKB:P31268",
  "term_id": "GO:0006357",
  "gene_symbol": "HOXA7"
}